quercitrin binding [GO:2001227] (molecular function) Sources: GOC:obol Definition: Binding to quercitrin. Relationships: is a type of GO:0043168; is a type of flavonoid binding [GO:0097243]; is_a GO:0097367